positive regulation of chaperone-mediated protein complex assembly [GO:0090035] (BP) Relationships: is_a positive regulation of protein-containing complex assembly [GO:0031334]; is a type of GO:0090034; RO_0002213 chaperone-mediated protein complex assembly [GO:0051131] Sources: GOC:BHF, GOC:dph, GOC:tb Definition: Any process that increases the frequency, rate, or extent of chaperone-mediated protein complex assembly. Chaperone-mediated protein complex assembly is the aggregation, arrangement and bonding together of a set of components to form a protein complex, mediated by chaperone molecules that do not form part of the finished complex.